{
  "gene_symbol": "KRT26",
  "gene_name": "Keratin, type I cytoskeletal 26",
  "term_label": "cytoskeleton",
  "term_id": "GO:0005856",
  "gene": "UniProtKB:Q7Z3Y9"
}